{
  "gene_symbol": "PHETA1",
  "term_label": "Unknown molecular function",
  "term_id": "UNKNOWN:0001",
  "gene_name": "Sesquipedalian-1",
  "gene": "UniProtKB:Q8N4B1"
}